{
  "gene_name": "Serine_threonine-protein phosphatase 4 regulatory subunit 3A",
  "term_label": "regulation of double-strand break repair",
  "term_id": "GO:2000779",
  "gene_symbol": "PPP4R3A",
  "gene": "UniProtKB:Q6IN85"
}